negative regulation of cytoplasmic pattern recognition receptor signaling pathway [GO:0039532] (biological process) Subtypes: GO:0034140, negative regulation of toll-like receptor 7 signaling pathway [GO:0034156], negative regulation of toll-like receptor 8 signaling pathway [GO:0034160], negative regulation of toll-like receptor 9 signaling pathway [GO:0034164], negative regulation of toll-like receptor 11 signaling pathway [GO:0034172], negative regulation of toll-like receptor 12 signaling pathway [GO:0034176], negative regulation of toll-like receptor 13 signaling pathway [GO:0034180], negative regulation of MDA-5 signaling pathway [GO:0039534], negative regulation of RIG-I signaling pathway [GO:0039536], negative regulation of nucleotide-binding domain, leucine rich repeat containing receptor signaling pathway [GO:0070425], negative regulation of inflammasome-mediated signaling pathway [GO:0141086], GO:0160049 Sources: GOC:bf, GOC:jl Relationships: is a type of negative regulation of immune system process [GO:0002683]; is a type of regulation of cytoplasmic pattern recognition receptor signaling pathway [GO:0039531]; is a type of GO:1902532; negatively regulates cytoplasmic pattern recognition receptor signaling pathway [GO:0002753] Also known as: negative regulation of cytosolic pattern recognition receptor signaling pathway, negative regulation of cytoplasmic pattern recognition receptor signaling pathway in response to virus, negative regulation of viral-induced cytoplasmic pattern recognition receptor signaling pathway, negative regulation of viral-induced cytoplasmic pattern recognition receptor signalling pathway, negative regulation of MAVS signaling Definition: Any process that stops, prevents, or reduces the frequency, rate or extent of the series of a cytoplasmic pattern recognition receptor signaling pathway.